{
  "gene_symbol": "IGHV7-4-1",
  "term_label": "Unknown cellular component",
  "gene_name": "Immunoglobulin heavy variable 7-4-1",
  "term_id": "UNKNOWN:0003",
  "gene": "UniProtKB:A0A0J9YVY3"
}